mitotic spindle checkpoint signaling [GO:0071174] (biological process) Definition: A signaling process that contributes to a mitotic cell cycle checkpoint that originates from the spindle and delays the metaphase/anaphase transition of a mitotic nuclear division until the spindle is correctly assembled and oriented, the completion of anaphase until chromosomes are attached to the spindle, or mitotic exit and cytokinesis when the spindle does not form. Sources: GOC:mtg_cell_cycle Also known as: mitotic cell cycle spindle checkpoint, mitotic spindle checkpoint, signal transduction involved in mitotic cell cycle spindle checkpoint, signal transduction involved in mitotic spindle checkpoint, topo II checkpoint, topoisomerase II checkpoint Note: Note that this term should not be used for direct manual annotation as it should always be possible to specify the type of spindle checkpoint (assembly, orientation checkpoints). Relationships: is a type of mitotic cell cycle checkpoint signaling [GO:0007093]; is a type of spindle checkpoint signaling [GO:0031577] Subtypes: mitotic spindle assembly checkpoint signaling [GO:0007094], mitotic spindle orientation checkpoint signaling [GO:0031578] Regulation: regulated by regulation of mitotic spindle checkpoint [GO:1903504]